negative regulation of secretion [GO:0051048] (biological process) Sources: GOC:ai Relationships: is a type of regulation of secretion [GO:0051046]; is a type of negative regulation of transport [GO:0051051]; negatively regulates GO:0046903 Also known as: down regulation of secretion, down-regulation of secretion, downregulation of secretion, inhibition of secretion Subtypes: negative regulation of peptide secretion [GO:0002792], negative regulation of gamma-aminobutyric acid secretion [GO:0014053], negative regulation of icosanoid secretion [GO:0032304], GO:0035814, negative regulation of gastric acid secretion [GO:0060455], negative regulation of mucus secretion [GO:0070256], GO:0090188, negative regulation of bile acid secretion [GO:0120190], negative regulation of lactation [GO:1903488], negative regulation of secretion by cell [GO:1903531], negative regulation of saliva secretion [GO:1905747], GO:2000293 Definition: Any process that stops, prevents, or reduces the frequency, rate or extent of the controlled release of a substance from a cell or a tissue.